estivation [GO:0042751] (biological process) Relationships: is a type of GO:0022611 Definition: Any process in which an organism enters and maintains a period of dormancy, similar to hibernation, but that occurs during the summer. It insulates against heat to prevent the harmful effects of the season. References: PMID:12443930 Sources: GOC:jl, Wikipedia:Estivation Also known as: aestivation